meristem initiation [GO:0010014] (biological process) Definition: Initiation of a region of tissue in a plant that is composed of one or more undifferentiated cells capable of undergoing mitosis and differentiation, thereby effecting growth and development of a plant by giving rise to more meristem or specialized tissue. Sources: GOC:sm Subtypes: embryonic meristem initiation [GO:0090421], axillary shoot meristem initiation [GO:0090506] Relationships: is a type of developmental process [GO:0032502]; is part of GO:0009933